{
  "gene_symbol": "IRX1",
  "gene": "UniProtKB:P78414",
  "term_id": "GO:0006357",
  "gene_name": "Iroquois-class homeodomain protein IRX-1",
  "term_label": "regulation of transcription by RNA polymerase II"
}